{
  "gene": "UniProtKB:Q96HA4",
  "term_id": "UNKNOWN:0002",
  "gene_name": "Uncharacterized protein C1orf159",
  "gene_symbol": "C1orf159",
  "term_label": "Unknown biological process"
}